regulation of CD8-positive, alpha-beta T cell proliferation [GO:2000564] (biological process) Relationships: is a type of GO:0046640; is a type of regulation of CD8-positive, alpha-beta T cell activation [GO:2001185]; regulates CD8-positive, alpha-beta T cell proliferation [GO:0035740] Sources: GOC:obol Subtypes: GO:2000565, positive regulation of CD8-positive, alpha-beta T cell proliferation [GO:2000566] Definition: Any process that modulates the frequency, rate or extent of CD8-positive, alpha-beta T cell proliferation.